miRNA metabolic process [GO:0010586] (biological process) Also known as: microRNA metabolic process Regulation: RO_0002211 by regulation of miRNA metabolic process [GO:2000628]; negatively regulated by negative regulation of miRNA metabolic process [GO:2000629]; positively regulated by positive regulation of miRNA metabolic process [GO:2000630] Definition: The chemical reactions and pathways involving miRNA, microRNA, a class of single-stranded RNA molecules of about 21-23 nucleotides in length, which regulates gene expression. Relationships: is a type of RNA metabolic process [GO:0016070] References: PMID:17993620 Subtypes: miRNA catabolic process [GO:0010587], GO:0061614